regulation of long-term synaptic potentiation [GO:1900271] (biological process) Definition: Any process that modulates the frequency, rate or extent of long-term synaptic potentiation. Sources: GOC:BHF, GOC:TermGenie Also known as: regulation of long-term potentiation, regulation of LTP Relationships: is a type of regulation of synaptic plasticity [GO:0048167]; regulates long-term synaptic potentiation [GO:0060291] Subtypes: GO:1900272, GO:1900273